{
  "gene_name": "C-type lectin domain family 12 member A",
  "term_id": "GO:0005886",
  "gene": "UniProtKB:Q5QGZ9",
  "term_label": "plasma membrane",
  "gene_symbol": "CLEC12A"
}